rhombomere development [GO:0021546] (biological process) Definition: The process whose specific outcome is the progression of the rhombomere over time, from its formation to the mature structure. Rhombomeres are transverse segments of the developing rhombencephalon. Rhombomeres are lineage restricted, express different genes from one another, and adopt different developmental fates. Subtypes: rhombomere 1 development [GO:0021567], rhombomere 2 development [GO:0021568], rhombomere 3 development [GO:0021569], rhombomere 4 development [GO:0021570], rhombomere 5 development [GO:0021571], rhombomere 6 development [GO:0021572], rhombomere 7 development [GO:0021573], rhombomere 8 development [GO:0021574] Sources: GOC:cls, GOC:dgh, GOC:dph, GOC:jid, GO_REF:0000021 Relationships: is a type of GO:0048856; is part of GO:0030902